{
  "term_label": "cytoplasm",
  "gene_symbol": "TRIM14",
  "gene": "UniProtKB:Q14142",
  "gene_name": "Tripartite motif-containing protein 14",
  "term_id": "GO:0005737"
}